{
  "term_id": "GO:0004252",
  "term_label": "serine-type endopeptidase activity",
  "gene_symbol": "PRSS58",
  "gene": "UniProtKB:Q8IYP2",
  "gene_name": "Serine protease 58"
}